plastoglobule [GO:0010287] (cellular component) Relationships: is a type of cellular anatomical structure [GO:0110165]; is part of chloroplast stroma [GO:0009570] References: PMID:16461379 Sources: GOC:tair_curators Also known as: PG, plastoglobuli Definition: A lipoprotein particle present in chloroplasts. They are rich in non-polar lipids (triglycerides, esters) as well as in prenylquinones, plastoquinone and tocopherols. Plastoglobules are often associated with thylakoid membranes, suggesting an exchange of lipids with thylakoids.